{
  "term_label": "Unknown biological process",
  "gene": "UniProtKB:A0A2R8Y747",
  "term_id": "UNKNOWN:0002",
  "gene_symbol": "A0A2R8Y747",
  "gene_name": "Uncharacterized protein"
}